{
  "gene_name": "Butyrophilin subfamily 3 member A2",
  "gene": "UniProtKB:P78410",
  "term_id": "GO:0009897",
  "gene_symbol": "BTN3A2",
  "term_label": "external side of plasma membrane"
}